{
  "term_id": "UNKNOWN:0001",
  "gene_name": "Cilia- and flagella-associated protein 69",
  "gene_symbol": "CFAP69",
  "term_label": "Unknown molecular function",
  "gene": "UniProtKB:A5D8W1"
}